{
  "gene_name": "Myosin regulatory light chain 2, ventricular_cardiac muscle isoform",
  "gene_symbol": "MYL2",
  "term_label": "myofibril",
  "term_id": "GO:0030016",
  "gene": "UniProtKB:P10916"
}